positive regulation of nutrient release by symbiont [GO:0052519] (BP) Sources: GOC:mtg_pamgo_17jul06 Relationships: is a type of modulation of nutrient release by symbiont [GO:0052460] Definition: Any process in which an organism activates, maintains or increases the frequency, rate or extent of the release of nutrients from a symbiont organism. The symbiont is defined as the smaller of the organisms involved in a symbiotic interaction. Also known as: positive regulation by host of nutrient release from symbiont, promotion of nutrient release from symbiont, up regulation by host of nutrient release from symbiont, up-regulation by host of nutrient release from symbiont, upregulation by host of nutrient release from symbiont, activation by host of nutrient release from symbiont, stimulation by host of nutrient release from symbiont